{
  "term_id": "GO:0005615",
  "term_label": "extracellular space",
  "gene_name": "Interleukin-8",
  "gene_symbol": "CXCL8",
  "gene": "UniProtKB:P10145"
}